{
  "gene_symbol": "CAMK2A",
  "term_id": "GO:0004683",
  "gene_name": "Calcium_calmodulin-dependent protein kinase type II subunit alpha",
  "term_label": "calcium/calmodulin-dependent protein kinase activity",
  "gene": "UniProtKB:Q9UQM7"
}